{
  "term_label": "Unknown cellular component",
  "term_id": "UNKNOWN:0003",
  "gene_symbol": "TEX29",
  "gene_name": "Testis-expressed protein 29",
  "gene": "UniProtKB:Q8N6K0"
}